{
  "term_label": "Unknown cellular component",
  "gene": "UniProtKB:Q9NVT9",
  "gene_symbol": "ARMC1",
  "gene_name": "Armadillo repeat-containing protein 1",
  "term_id": "UNKNOWN:0003"
}